{
  "term_id": "GO:0001817",
  "gene_symbol": "VTCN1",
  "gene": "UniProtKB:Q7Z7D3",
  "term_label": "regulation of cytokine production",
  "gene_name": "V-set domain-containing T-cell activation inhibitor 1"
}